ectodermal cell fate determination [GO:0001713] (biological process) Definition: The cell fate determination process that results in a cell becoming capable of differentiating autonomously into an ectoderm cell regardless of its environment; upon determination, the cell fate cannot be reversed. Relationships: is a type of cell fate determination [GO:0001709]; is part of ectodermal cell fate commitment [GO:0001712] Also known as: ectoderm cell fate determination Sources: GOC:go_curators, ISBN:0878932437